{
  "term_label": "Unknown biological process",
  "term_id": "UNKNOWN:0002",
  "gene": "UniProtKB:Q03395",
  "gene_symbol": "ROM1",
  "gene_name": "Rod outer segment membrane protein 1"
}